{
  "gene_name": "Ribosomal oxygenase 1",
  "gene": "UniProtKB:Q9H6W3",
  "term_id": "UNKNOWN:0002",
  "gene_symbol": "RIOX1",
  "term_label": "Unknown biological process"
}